negative regulation of DNA-templated transcription [GO:0045892] (biological process) Definition: Any process that stops, prevents, or reduces the frequency, rate or extent of cellular DNA-templated transcription. Sources: GOC:go_curators, GOC:txnOH Also known as: down regulation of transcription, DNA-dependent, down-regulation of transcription, DNA-dependent, downregulation of transcription, DNA-dependent, negative regulation of cellular transcription, DNA-dependent, negative regulation of transcription, DNA-dependent, negative regulation of transcription, DNA-templated, inhibition of transcription, DNA-dependent, down regulation of gene-specific transcription, down-regulation of gene-specific transcription, downregulation of gene-specific transcription, inhibition of gene-specific transcription, negative regulation of gene-specific transcription, transcription repressor activity Relationships: is a type of regulation of DNA-templated transcription [GO:0006355]; is a type of GO:1902679; negatively regulates DNA-templated transcription [GO:0006351] Subtypes: GO:0000122, negative regulation of transcription by transcription factor catabolism [GO:0010620], negative regulation of transcription by competitive promoter binding [GO:0010944], GO:0016479, negative regulation of transcription by RNA polymerase III [GO:0016480], negative regulation of DNA-templated transcription, elongation [GO:0032785], carbon catabolite repression of transcription [GO:0045013], GO:0045894, GO:0060195, GO:0060567, nitrogen catabolite repression of transcription [GO:0090295], negative regulation of lncRNA transcription [GO:0140744], negative regulation of mitochondrial transcription [GO:0170070], GO:1902894, negative regulation of transcription by RNA polymerase V [GO:1904280], negative regulation of DNA-templated transcription initiation [GO:2000143]